positive regulation of cumulus cell differentiation [GO:0045594] (biological process) Relationships: is a type of positive regulation of epithelial cell differentiation [GO:0030858]; is a type of regulation of cumulus cell differentiation [GO:0045592]; is a type of positive regulation of reproductive process [GO:2000243]; positively regulates cumulus cell differentiation [GO:0001549] Sources: GOC:go_curators Definition: Any process that activates or increases the frequency, rate or extent of ovarian cumulus cell differentiation. Also known as: positive regulation of ovarian cumulus cell differentiation, up regulation of cumulus cell differentiation, up-regulation of cumulus cell differentiation, upregulation of cumulus cell differentiation, activation of cumulus cell differentiation, stimulation of cumulus cell differentiation